{
  "gene": "UniProtKB:Q96B01",
  "gene_symbol": "RAD51AP1",
  "term_id": "GO:0036297",
  "gene_name": "RAD51-associated protein 1",
  "term_label": "interstrand cross-link repair"
}